glycolipid metabolic process [GO:0006664] (biological process) Sources: ISBN:0198547684 Relationships: is a type of GO:0006643; is_a liposaccharide metabolic process [GO:1903509] Subtypes: GPI anchor metabolic process [GO:0006505], GO:0006687, GO:0009247, galactolipid metabolic process [GO:0019374], GO:0019377, GO:0046493 Also known as: glycolipid metabolism Definition: The chemical reactions and pathways involving glycolipids, a class of 1,2-di-O-acylglycerols joined at oxygen 3 by a glycosidic linkage to a carbohydrate part (usually a mono-, di- or tri-saccharide). Some substances classified as bacterial glycolipids have the sugar group acylated by one or more fatty acids and the glycerol group may be absent.